regulation of nodal receptor complex assembly [GO:1900123] (biological process) Also known as: regulation of ActRIIB.ALK4.EGF-CFC complex formation, regulation of nodal receptor complex formation Subtypes: GO:1900124 Relationships: is a type of regulation of protein-containing complex assembly [GO:0043254]; regulates nodal receptor complex assembly [GO:0038099] References: PMID:15062104 Sources: GOC:TermGenie, GOC:signaling Definition: Any process that modulates the frequency, rate or extent of nodal receptor complex assembly.